{
  "gene_name": "Netrin receptor UNC5B",
  "term_label": "Unknown cellular component",
  "gene": "UniProtKB:Q8IZJ1",
  "gene_symbol": "UNC5B",
  "term_id": "UNKNOWN:0003"
}